{
  "gene_name": "ADP-ribosylation factor 5",
  "gene": "UniProtKB:P84085",
  "term_id": "GO:0005886",
  "gene_symbol": "ARF5",
  "term_label": "plasma membrane"
}